{
  "gene_symbol": "TOR2A",
  "gene_name": "Torsin-2A",
  "gene": "UniProtKB:Q5JU69",
  "term_label": "nuclear envelope",
  "term_id": "GO:0005635"
}